high molecular weight kininogen receptor complex [GO:0030988] (cellular component) Definition: A protein complex that acts as a receptor for high molecular weight kininogens. In humans, this receptor includes the CK1 and uPAR proteins. References: PMID:11290596 Sources: GOC:mah Relationships: is a type of plasma membrane signaling receptor complex [GO:0098802]